maltose transport complex [GO:1990060] (cellular component) Definition: Protein complex facilitating ATP-dependent maltose transport through inner cell membrane (periplasm to cytoplasm) in Gram-negative bacteria. In E. coli the system is composed of a periplasmic maltose-binding protein (MBP), two integral membrane proteins, MalF and MalG, and two copies of the cytoplasmic ATP-binding cassette MalK. References: PMID:18033289 Also known as: maltose ABC transporter complex, maltose ATP-binding cassette transporter complex Relationships: is a type of ATP-binding cassette (ABC) transporter complex [GO:0043190]